regulation of mesenchymal cell apoptotic process involved in mesonephric nephron morphogenesis [GO:0061295] (biological process) Also known as: regulation of mesenchymal stem cell apoptotic process involved in mesonephric nephron morphogenesis, regulation of mesenchymal stem cell apoptosis involved in mesonephric nephron morphogenesis Subtypes: negative regulation of mesenchymal cell apoptotic process involved in mesonephric nephron morphogenesis [GO:0061296], GO:0061297 Definition: Any process that modulates the occurrence or rate of mesenchymal stem cell death by apoptotic process that contributes to the shaping of the nephron in the mesonephros. Sources: GOC:mtg_apoptosis, GOC:mtg_kidney_jan10 Relationships: is a type of GO:0072039; regulates GO:0061235; regulates mesenchymal cell apoptotic process involved in mesonephric nephron morphogenesis [GO:1901146]